{
  "gene": "UniProtKB:Q8WTW4",
  "term_label": "cellular response to amino acid starvation",
  "gene_name": "GATOR complex protein NPRL2",
  "gene_symbol": "NPRL2",
  "term_id": "GO:0034198"
}